nucleotide-excision repair, DNA gap filling [GO:0006297] (biological process) Relationships: is_a DNA metabolic process [GO:0006259]; is part of nucleotide-excision repair [GO:0006289] Sources: ISBN:0815316194 Definition: Repair of the gap in the DNA helix by DNA polymerase and DNA ligase after the portion of the strand containing the lesion has been removed by pyrimidine-dimer repair enzymes.